{
  "gene_name": "Cytoplasmic dynein 1 intermediate chain 2",
  "gene": "UniProtKB:Q13409",
  "term_label": "dynein light chain binding",
  "term_id": "GO:0045503",
  "gene_symbol": "DYNC1I2"
}